{
  "gene": "UniProtKB:Q86YI8",
  "gene_symbol": "PHF13",
  "gene_name": "PHD finger protein 13",
  "term_label": "chromatin binding",
  "term_id": "GO:0003682"
}